{
  "gene_name": "Histone-lysine N-methyltransferase SMYD3",
  "term_id": "GO:0005634",
  "gene": "UniProtKB:Q9H7B4",
  "gene_symbol": "SMYD3",
  "term_label": "nucleus"
}